{
  "gene_symbol": "NLGN3",
  "gene": "UniProtKB:Q9NZ94",
  "term_label": "presynaptic membrane assembly",
  "term_id": "GO:0097105",
  "gene_name": "Neuroligin-3"
}